{
  "gene": "UniProtKB:O75752",
  "gene_name": "UDP-GalNAc:beta-1,3-N-acetylgalactosaminyltransferase 1",
  "term_id": "GO:0000139",
  "gene_symbol": "B3GALNT1",
  "term_label": "Golgi membrane"
}